acid-CoA ligase (GDP-forming) activity [GO:0047612] (molecular function) Also known as: acid:CoA ligase (GDP-forming), acyl coenzyme A synthetase (guanosine diphosphate forming), acyl-CoA synthetase (GDP-forming) activity Definition: Catalysis of the reaction: a carboxylate + CoA + GTP = acyl-CoA + GDP + H+ + phosphate. Relationships: is a type of acid-thiol ligase activity [GO:0016878] Sources: RHEA:10968